{
  "gene_name": "Myelin-associated glycoprotein",
  "gene": "UniProtKB:P20916",
  "term_id": "GO:0007155",
  "term_label": "cell adhesion",
  "gene_symbol": "MAG"
}